{
  "gene": "UniProtKB:Q5TC79",
  "gene_symbol": "ZBTB37",
  "gene_name": "Zinc finger and BTB domain-containing protein 37",
  "term_label": "negative regulation of transcription by RNA polymerase II",
  "term_id": "GO:0000122"
}